spermidine:caffeoyl CoA N-acyltransferase activity [GO:0080074] (molecular function) References: PMID:19077165 Definition: Catalysis of the transfer of a caffeoyl group to a nitrogen atom on the spermidine molecule. Relationships: is a type of N-acyltransferase activity [GO:0016410]